{
  "gene_name": "Putative zinc finger protein 66",
  "term_id": "GO:0000978",
  "term_label": "RNA polymerase II cis-regulatory region sequence-specific DNA binding",
  "gene": "UniProtKB:Q6ZN08",
  "gene_symbol": "ZNF66"
}